{
  "term_label": "glutathione metabolic process",
  "gene_name": "Glutathione S-transferase kappa 1",
  "gene": "UniProtKB:Q9Y2Q3",
  "term_id": "GO:0006749",
  "gene_symbol": "GSTK1"
}